{
  "term_id": "GO:0000139",
  "gene_symbol": "SLC35B1",
  "gene": "UniProtKB:P78383",
  "term_label": "Golgi membrane",
  "gene_name": "Solute carrier family 35 member B1"
}